endoplasmic reticulum cisternal network [GO:0071781] (cellular component) References: PMID:16469703, PMID:20434336 Sources: GOC:vw Relationships: is a type of endoplasmic reticulum subcompartment [GO:0098827] Also known as: ER cisternal network Definition: A subcompartment of the endoplasmic reticulum consisting of flattened, disc-shaped domains known as cisternae. These are typically found close to the nucleus and are generally more prominent in secretory cells.